{
  "gene": "UniProtKB:Q05195",
  "term_label": "Unknown cellular component",
  "term_id": "UNKNOWN:0003",
  "gene_symbol": "MXD1",
  "gene_name": "Max dimerization protein 1"
}